{
  "term_id": "GO:0005634",
  "gene": "UniProtKB:Q16667",
  "term_label": "nucleus",
  "gene_symbol": "CDKN3",
  "gene_name": "Cyclin-dependent kinase inhibitor 3"
}